{
  "term_label": "proteasome regulatory particle, base subcomplex",
  "gene_name": "26S proteasome regulatory subunit 8",
  "gene": "UniProtKB:P62195",
  "gene_symbol": "PSMC5",
  "term_id": "GO:0008540"
}